proton-transporting V-type ATPase, V0 domain [GO:0033179] (cellular component) Definition: A protein complex that forms part of a proton-transporting V-type ATPase and mediates proton transport across a membrane. The V0 complex consists of at least four different subunits (a,c,d and e); six or more c subunits form a proton-binding rotor ring. Relationships: is a type of proton-transporting two-sector ATPase complex, proton-transporting domain [GO:0033177]; is part of proton-transporting V-type ATPase complex [GO:0033176] Subtypes: GO:0000220, plasma membrane proton-transporting V-type ATPase, V0 domain [GO:0000222] References: PMID:16449553 Sources: GOC:mah, ISBN:0716743663